IgY immunoglobulin complex [GO:0071760] (cellular component) Note: Note that an IgY immunoglobulin complex has the function of antigen binding if a suitable antigen is available. Note that IgY is found in amphibians, reptiles, and birds. Relationships: is a type of immunoglobulin complex [GO:0019814] Definition: A protein complex composed of two identical immunoglobulin heavy chains of the IgY isotype and two identical immunoglobulin light chains, held together by disulfide bonds. An IgY immunoglobulin complex may be embedded in the plasma membrane or present in the extracellular space, in mucosal areas or other tissues, or circulating in the blood or lymph. Sources: GOC:add, ISBN:0781765196